{
  "gene": "UniProtKB:Q7Z5Q1",
  "term_id": "GO:0043022",
  "term_label": "ribosome binding",
  "gene_symbol": "CPEB2",
  "gene_name": "Cytoplasmic polyadenylation element-binding protein 2"
}